negative regulation of selenocysteine incorporation [GO:1904570] (biological process) Also known as: down regulation of selenocysteine incorporation, down-regulation of selenocysteine incorporation, downregulation of selenocysteine incorporation, inhibition of selenocysteine incorporation References: PMID:21685449 Sources: GOC:TermGenie, GO_REF:0000058 Relationships: is_a negative regulation of translational elongation [GO:0045900]; is_a regulation of selenocysteine incorporation [GO:1904569]; negatively regulates GO:0001514 Definition: Any process that stops, prevents or reduces the frequency, rate or extent of selenocysteine incorporation.